{
  "gene_symbol": "SSU72L5",
  "gene_name": "RNA polymerase II subunit A C-terminal domain phosphatase SSU72 like protein 5",
  "gene": "UniProtKB:A0A1W2PQ64",
  "term_label": "mRNA cleavage and polyadenylation specificity factor complex",
  "term_id": "GO:0005847"
}